{
  "gene_name": "Putative uncharacterized protein FLJ46214",
  "gene_symbol": "Q6ZRN7",
  "term_label": "Unknown biological process",
  "term_id": "UNKNOWN:0002",
  "gene": "UniProtKB:Q6ZRN7"
}